positive regulation of the force of heart contraction by neuronal norepinephrine [GO:0003110] (biological process) Definition: The process in which the release of norepinephrine from nerve endings modulates the force of heart muscle contraction. Sources: GOC:mtg_cardio Relationships: is a type of positive regulation of the force of heart contraction by norepinephrine [GO:0003061] Also known as: increased force of heart contraction by neuronal norepinephrine, increased force of heart contraction by neuronal noradrenaline